{
  "term_id": "GO:0005761",
  "gene_name": "Large ribosomal subunit protein mL48",
  "gene": "UniProtKB:Q96GC5",
  "gene_symbol": "MRPL48",
  "term_label": "mitochondrial ribosome"
}